positive regulation of protein export from nucleus during meiotic anaphase II [GO:1900199] (biological process) Relationships: is a type of positive regulation of protein export from nucleus [GO:0046827]; happens during meiotic anaphase II [GO:0007138] References: PMID:20970342 Sources: GOC:TermGenie, GOC:al Definition: Any process that activates or increases the frequency, rate or extent of directed movement of proteins from the nucleus into the cytoplasm, during anaphase occurring as part of meiosis II. Also known as: positive regulation of protein export from nucleus involved in meiotic anaphase II